{
  "term_id": "UNKNOWN:0002",
  "gene_name": "Complement C1q tumor necrosis factor-related protein 7",
  "term_label": "Unknown biological process",
  "gene": "UniProtKB:Q9BXJ2",
  "gene_symbol": "C1QTNF7"
}